mitochondrial translational elongation [GO:0070125] (biological process) Sources: GOC:mah Relationships: is a type of translational elongation [GO:0006414]; is part of GO:0032543; occurs in mitochondrion [GO:0005739] Regulation: regulated by regulation of mitochondrial translational elongation [GO:1905082]; negatively regulated by negative regulation of mitochondrial translational elongation [GO:1905083]; positively regulated by positive regulation of mitochondrial translational elongation [GO:1905084] Definition: The successive addition of amino acid residues to a nascent polypeptide chain during protein biosynthesis in a mitochondrion. Also known as: mitochondrial translation elongation